{
  "gene_symbol": "LIMK2",
  "term_id": "GO:0005634",
  "term_label": "nucleus",
  "gene_name": "LIM domain kinase 2",
  "gene": "UniProtKB:P53671"
}